{
  "gene_symbol": "PRR9",
  "term_label": "Unknown molecular function",
  "term_id": "UNKNOWN:0001",
  "gene_name": "Proline-rich protein 9",
  "gene": "UniProtKB:Q5T870"
}